{
  "term_label": "mitochondrion",
  "term_id": "GO:0005739",
  "gene": "UniProtKB:Q96B49",
  "gene_symbol": "TOMM6",
  "gene_name": "Mitochondrial import receptor subunit TOM6 homolog"
}